protein-pyridoxal-5-phosphate linkage [GO:0018352] (biological process) Sources: GOC:mah Regulation: regulated by regulation of protein-pyridoxal-5-phosphate linkage [GO:1904285]; negatively regulated by negative regulation of protein-pyridoxal-5-phosphate linkage [GO:1904286]; positively regulated by positive regulation of protein-pyridoxal-5-phosphate linkage [GO:1904287] Definition: The formation of a linkage between a protein amino acid and pyridoxal-5-phosphate. Subtypes: protein-pyridoxal-5-phosphate linkage via peptidyl-N6-pyridoxal phosphate-L-lysine [GO:0018272] Relationships: is a type of protein modification process [GO:0036211]